{
  "gene_name": "Membrane primary amine oxidase",
  "term_label": "plasma membrane",
  "gene": "UniProtKB:Q16853",
  "term_id": "GO:0005886",
  "gene_symbol": "AOC3"
}